{
  "gene_symbol": "CXXC4",
  "gene": "UniProtKB:Q9H2H0",
  "term_label": "methyl-CpG binding",
  "term_id": "GO:0008327",
  "gene_name": "CXXC-type zinc finger protein 4"
}